{
  "term_id": "UNKNOWN:0001",
  "gene_name": "Zinc finger protein 26",
  "gene": "UniProtKB:P17031",
  "term_label": "Unknown molecular function",
  "gene_symbol": "ZNF26"
}